{
  "gene_name": "Actin-like protein 10",
  "gene_symbol": "ACTL10",
  "term_id": "UNKNOWN:0002",
  "term_label": "Unknown biological process",
  "gene": "UniProtKB:Q5JWF8"
}